{
  "term_id": "GO:0031647",
  "gene_symbol": "USP30",
  "gene_name": "Ubiquitin carboxyl-terminal hydrolase 30",
  "term_label": "regulation of protein stability",
  "gene": "UniProtKB:Q70CQ3"
}